positive regulation of ossification [GO:0045778] (biological process) Definition: Any process that activates or increases the frequency, rate or extent of ossification, the formation of bone or of a bony substance or the conversion of fibrous tissue or of cartilage into bone or a bony substance. Also known as: positive regulation of bone biosynthesis, positive regulation of bone formation, up regulation of ossification, up-regulation of ossification, upregulation of ossification, activation of ossification, stimulation of ossification Relationships: is a type of regulation of ossification [GO:0030278]; is a type of positive regulation of multicellular organismal process [GO:0051240]; positively regulates GO:0001503 Subtypes: positive regulation of bone mineralization [GO:0030501] Sources: GOC:go_curators